{
  "gene_symbol": "CFAP47",
  "gene_name": "Cilia- and flagella-associated protein 47",
  "gene": "UniProtKB:Q6ZTR5",
  "term_label": "Unknown molecular function",
  "term_id": "UNKNOWN:0001"
}